toluene oxidation [GO:0019600] (biological process) Sources: GOC:mah Relationships: is_a toluene metabolic process [GO:0018970] Definition: The chemical reactions and pathways resulting in the loss of electrons from one or more atoms in toluene. Subtypes: toluene oxidation via 2-hydroxytoluene [GO:0019601], toluene oxidation via 3-hydroxytoluene [GO:0019602], toluene oxidation via 4-hydroxytoluene [GO:0019603], toluene oxidation to catechol [GO:0019604], toluene oxidation via toluene-cis-1,2-dihydrodiol [GO:0019696]